{
  "term_id": "GO:0009617",
  "term_label": "response to bacterium",
  "gene_name": "T cell receptor alpha variable 26-2",
  "gene": "UniProtKB:A0A0B4J265",
  "gene_symbol": "TRAV26-2"
}